verruculogen biosynthetic process [GO:1902181] (biological process) References: PMID:23649274 Sources: GOC:TermGenie, GOC:di Relationships: is a type of diol biosynthetic process [GO:0034312]; is a type of indole alkaloid biosynthetic process [GO:0035835]; is a type of GO:1901503 Also known as: verruculogen anabolism, verruculogen biosynthesis, verruculogen formation, verruculogen synthesis Definition: The chemical reactions and pathways resulting in the formation of verruculogen.